CCR5 chemokine receptor binding [GO:0031730] (molecular function) Also known as: CCR5 chemokine receptor ligand Relationships: is a type of CCR chemokine receptor binding [GO:0048020] Sources: GOC:mah, GOC:nln Definition: Binding to a CCR5 chemokine receptor.